{
  "gene_symbol": "KRTAP10-12",
  "gene_name": "Keratin-associated protein 10-12",
  "term_id": "UNKNOWN:0003",
  "term_label": "Unknown cellular component",
  "gene": "UniProtKB:P60413"
}